regulation of Schwann cell proliferation involved in axon regeneration [GO:1905044] (biological process) Subtypes: GO:1905045, positive regulation of Schwann cell proliferation involved in axon regeneration [GO:1905046] Relationships: is a type of regulation of Schwann cell proliferation [GO:0010624]; regulates GO:0014011 Definition: Any process that modulates the frequency, rate or extent of Schwann cell proliferation involved in axon regeneration. References: PMID:22393241 Sources: GOC:BHF, GOC:BHF_miRNA, GOC:TermGenie, GOC:rph, GO_REF:0000058